{
  "gene_name": "SID1 transmembrane family member 2",
  "gene": "UniProtKB:Q8NBJ9",
  "gene_symbol": "SIDT2",
  "term_label": "plasma membrane",
  "term_id": "GO:0005886"
}